{
  "gene_symbol": "CFHR4",
  "term_id": "GO:0001851",
  "gene_name": "Complement factor H-related protein 4",
  "term_label": "complement component C3b binding",
  "gene": "UniProtKB:Q92496"
}